{
  "gene_symbol": "OPTC",
  "gene_name": "Opticin",
  "term_id": "GO:0030199",
  "gene": "UniProtKB:Q9UBM4",
  "term_label": "collagen fibril organization"
}